{
  "gene": "UniProtKB:P83859",
  "gene_symbol": "QRFP",
  "gene_name": "Orexigenic neuropeptide QRFP",
  "term_label": "neuropeptide signaling pathway",
  "term_id": "GO:0007218"
}